{
  "gene": "UniProtKB:P50221",
  "gene_name": "Homeobox protein MOX-1",
  "term_label": "RNA polymerase II cis-regulatory region sequence-specific DNA binding",
  "term_id": "GO:0000978",
  "gene_symbol": "MEOX1"
}